{
  "gene_symbol": "RBBP6",
  "gene": "UniProtKB:Q7Z6E9",
  "gene_name": "E3 ubiquitin-protein ligase RBBP6",
  "term_label": "nucleus",
  "term_id": "GO:0005634"
}